{
  "term_id": "GO:0006367",
  "gene_name": "Transcription initiation factor IIE subunit beta",
  "gene": "UniProtKB:P29084",
  "term_label": "transcription initiation at RNA polymerase II promoter",
  "gene_symbol": "GTF2E2"
}